{
  "gene_name": "5-hydroxytryptamine receptor 2A",
  "term_label": "dendrite",
  "term_id": "GO:0030425",
  "gene_symbol": "HTR2A",
  "gene": "UniProtKB:P28223"
}